{
  "gene_symbol": "RUSC1-AS1",
  "gene": "UniProtKB:Q66K80",
  "term_id": "UNKNOWN:0002",
  "term_label": "Unknown biological process",
  "gene_name": "Putative uncharacterized protein RUSC1-AS1"
}